positive regulation of platelet activation [GO:0010572] (BP) Sources: GOC:dph, GOC:sl, GOC:tb Relationships: is a type of regulation of platelet activation [GO:0010543]; is a type of GO:0050867; positively regulates platelet activation [GO:0030168] Definition: Any process that increases the rate or frequency of platelet activation. Platelet activation is a series of progressive, overlapping events triggered by exposure of the platelets to subendothelial tissue.